{
  "term_label": "protein-macromolecule adaptor activity",
  "gene": "UniProtKB:Q9NRL3",
  "gene_symbol": "STRN4",
  "term_id": "GO:0030674",
  "gene_name": "Striatin-4"
}